{
  "term_id": "GO:0048787",
  "gene_symbol": "LRFN3",
  "gene": "UniProtKB:Q9BTN0",
  "term_label": "presynaptic active zone membrane",
  "gene_name": "Leucine-rich repeat and fibronectin type-III domain-containing protein 3"
}